{
  "gene_name": "TBC1 domain family member 3B",
  "gene": "UniProtKB:A6NDS4",
  "gene_symbol": "TBC1D3B",
  "term_label": "Unknown cellular component",
  "term_id": "UNKNOWN:0003"
}